non-sequence-specific DNA binding, bending [GO:0044378] (molecular function) Relationships: is a type of DNA binding, bending [GO:0008301] Definition: The activity of binding selectively and non-covalently to DNA in a sequence-independent manner and distorting the original structure of DNA, typically a straight helix, into a bend, or increasing the bend if the original structure was intrinsically bent due to its sequence. References: PMID:20123079 Sources: GOC:jl, GOC:vw Also known as: DNA bending involving non-sequence-specific DNA binding